{
  "term_id": "GO:0006729",
  "gene": "UniProtKB:P35270",
  "term_label": "tetrahydrobiopterin biosynthetic process",
  "gene_name": "Sepiapterin reductase",
  "gene_symbol": "SPR"
}